{
  "gene_symbol": "ZNF783",
  "term_label": "regulation of DNA-templated transcription",
  "term_id": "GO:0006355",
  "gene_name": "Zinc finger protein 783",
  "gene": "UniProtKB:Q6ZMS7"
}